{
  "gene_name": "Integrator complex subunit 15",
  "gene": "UniProtKB:Q96N11",
  "gene_symbol": "INTS15",
  "term_id": "UNKNOWN:0001",
  "term_label": "Unknown molecular function"
}